{
  "term_id": "GO:0060158",
  "gene_symbol": "GNA14",
  "gene": "UniProtKB:O95837",
  "term_label": "phospholipase C-activating dopamine receptor signaling pathway",
  "gene_name": "Guanine nucleotide-binding protein subunit alpha-14"
}